{
  "gene_symbol": "HYPK",
  "term_id": "UNKNOWN:0003",
  "gene": "UniProtKB:Q9NX55",
  "gene_name": "Huntingtin-interacting protein K",
  "term_label": "Unknown cellular component"
}